{
  "term_label": "central nervous system development",
  "term_id": "GO:0007417",
  "gene_name": "Amyloid-beta precursor protein",
  "gene_symbol": "APP",
  "gene": "UniProtKB:P05067"
}